{
  "gene_name": "DNA damage-inducible transcript 3 protein",
  "gene": "UniProtKB:P35638",
  "term_id": "GO:0000122",
  "term_label": "negative regulation of transcription by RNA polymerase II",
  "gene_symbol": "DDIT3"
}